{
  "gene": "UniProtKB:Q9Y234",
  "term_id": "GO:0005739",
  "gene_symbol": "LIPT1",
  "gene_name": "Lipoyltransferase 1, mitochondrial",
  "term_label": "mitochondrion"
}